{
  "gene": "UniProtKB:O43240",
  "term_label": "secretory granule",
  "term_id": "GO:0030141",
  "gene_symbol": "KLK10",
  "gene_name": "Kallikrein-10"
}